{
  "term_id": "UNKNOWN:0003",
  "gene_name": "Beta-klotho",
  "term_label": "Unknown cellular component",
  "gene": "UniProtKB:Q86Z14",
  "gene_symbol": "KLB"
}